diferric-transferrin reductase (NAD+) activity [GO:0047852] (MF) Definition: Catalysis of the reaction: transferrin[Fe2+]2 + NAD+ = transferrin[Fe3+]2 + NADH. Also known as: NADH diferric transferrin reductase activity, diferric transferrin reductase activity, transferrin reductase activity, transferrin[Fe(II)]2:NAD+ oxidoreductase activity Relationships: is a type of oxidoreductase activity, acting on metal ions, NAD or NADP as acceptor [GO:0016723] Sources: RHEA:13841